{
  "gene_symbol": "SANBR",
  "gene_name": "SANT and BTB domain regulator of class switch recombination",
  "term_label": "Unknown cellular component",
  "gene": "UniProtKB:Q6NSI8",
  "term_id": "UNKNOWN:0003"
}